appressorium maturation [GO:0075035] (BP) Sources: GOC:pamgo_curators Relationships: is a type of formation of structure involved in a symbiotic process [GO:0044111]; is part of appressorium formation [GO:0075016] Definition: The process in which specialized features of the symbiont appressorium are acquired post initiation, to aid in infection of the host. The host is defined as the larger of the organisms involved in a symbiotic interaction. Also known as: appressorium maturation on or near host, maturation of symbiont appressorium on or near host, maturation of appressorium on or near host